{
  "gene_symbol": "CAV3",
  "term_id": "GO:0042383",
  "term_label": "sarcolemma",
  "gene": "UniProtKB:P56539",
  "gene_name": "Caveolin-3"
}